dGTP binding [GO:0032567] (molecular function) Sources: GOC:mah Definition: Binding to dGTP, deoxyguanosine triphosphate. Relationships: is a type of GO:0032560; is a type of anion binding [GO:0043168]